{
  "gene_symbol": "LYPD3",
  "gene": "UniProtKB:O95274",
  "term_id": "UNKNOWN:0002",
  "term_label": "Unknown biological process",
  "gene_name": "Ly6_PLAUR domain-containing protein 3"
}